{
  "gene_symbol": "TMEM262",
  "gene_name": "Cation channel sperm-associated auxiliary subunit TMEM262",
  "term_id": "UNKNOWN:0003",
  "term_label": "Unknown cellular component",
  "gene": "UniProtKB:E9PQX1"
}